ELYC domain binding [GO:0090542] (molecular function) References: PMID:18032582, PMID:19525971 Sources: GOC:pm Definition: Binding to a ELYC protein domain. The ELYC domain is an approximately 150 amino acid sequence which contains a highly conserved tetrapeptide sequence, ELYC. Relationships: is a type of protein domain specific binding [GO:0019904]